terminal cisterna lumen [GO:0014804] (cellular component) Sources: GOC:mtg_muscle Relationships: is a type of sarcoplasmic reticulum lumen [GO:0033018]; is part of GO:0014802 Definition: The region between the inner and outer lipid bilayers of the terminal cisterna envelope. This space is enriched in calsequestrin.